open tracheal system development [GO:0007424] (biological process) Relationships: is a type of GO:0060541 References: PMID:8625828 Sources: GOC:mtg_sensu Note: See also the fly_anatomy.ontology term 'tracheal system ; FBbt:00005024'. Definition: The process whose specific outcome is the progression of an open tracheal system over time, from its formation to the mature structure. An open tracheal system is a respiratory system, a branched network of epithelial tubes that supplies oxygen to target tissues via spiracles. An example of this is found in Drosophila melanogaster.